establishment of epithelial cell planar polarity [GO:0090163] (biological process) Relationships: is a type of establishment of epithelial cell polarity [GO:0090162] Definition: The specification and formation of the polarity of an epithelial cell along the plane of the epithelial tissue. Sources: GOC:ascb_2009, GOC:dph, GOC:tb